{
  "gene_symbol": "RBM44",
  "term_id": "GO:0071013",
  "gene_name": "RNA-binding protein 44",
  "gene": "UniProtKB:Q6ZP01",
  "term_label": "catalytic step 2 spliceosome"
}